{
  "gene": "UniProtKB:P50748",
  "gene_name": "Kinetochore-associated protein 1",
  "gene_symbol": "KNTC1",
  "term_id": "GO:0000070",
  "term_label": "mitotic sister chromatid segregation"
}